{
  "gene": "UniProtKB:P05787",
  "term_id": "UNKNOWN:0001",
  "gene_symbol": "KRT8",
  "term_label": "Unknown molecular function",
  "gene_name": "Keratin, type II cytoskeletal 8"
}